{
  "term_label": "monoacylglycerol lipase activity",
  "gene": "UniProtKB:Q96SE0",
  "term_id": "GO:0047372",
  "gene_name": "Protein ABHD1",
  "gene_symbol": "ABHD1"
}